myoinhibitory hormone activity [GO:0016085] (molecular function) References: PMID:8902848 Sources: GOC:mah Relationships: is a type of hormone activity [GO:0005179] Definition: The action characteristic of myostimulatory hormone, a peptide hormone that inhibits muscle contraction.